{
  "term_id": "GO:0005634",
  "term_label": "nucleus",
  "gene_symbol": "KLHL31",
  "gene_name": "Kelch-like protein 31",
  "gene": "UniProtKB:Q9H511"
}